{
  "gene_symbol": "NIN",
  "gene_name": "Ninein",
  "term_id": "GO:0005814",
  "gene": "UniProtKB:Q8N4C6",
  "term_label": "centriole"
}